{
  "gene_symbol": "KIR2DS5",
  "term_label": "plasma membrane",
  "gene_name": "Killer cell immunoglobulin-like receptor 2DS5",
  "gene": "UniProtKB:Q14953",
  "term_id": "GO:0005886"
}